{
  "term_label": "gap junction-mediated intercellular transport",
  "gene_symbol": "GJB2",
  "term_id": "GO:1990349",
  "gene_name": "Gap junction beta-2 protein",
  "gene": "UniProtKB:P29033"
}